{
  "gene": "UniProtKB:P15313",
  "gene_name": "V-type proton ATPase subunit B, kidney isoform",
  "term_label": "proton transmembrane transport",
  "gene_symbol": "ATP6V1B1",
  "term_id": "GO:1902600"
}